{
  "gene_name": "Membrane-associated phosphatidylinositol transfer protein 2",
  "term_label": "phosphatidylcholine binding",
  "gene": "UniProtKB:Q9BZ72",
  "term_id": "GO:0031210",
  "gene_symbol": "PITPNM2"
}